{
  "gene_name": "Cilia- and flagella-associated protein 36",
  "term_label": "axoneme",
  "term_id": "GO:0005930",
  "gene_symbol": "CFAP36",
  "gene": "UniProtKB:Q96G28"
}